{
  "term_label": "Unknown biological process",
  "gene_symbol": "C21orf140",
  "gene_name": "Uncharacterized protein C21orf140",
  "term_id": "UNKNOWN:0002",
  "gene": "UniProtKB:B9A014"
}